{
  "term_label": "nucleus",
  "gene": "UniProtKB:Q9Y222",
  "gene_name": "Cyclin-D-binding Myb-like transcription factor 1",
  "term_id": "GO:0005634",
  "gene_symbol": "DMTF1"
}